{
  "gene_symbol": "GP1BB",
  "gene_name": "Platelet glycoprotein Ib beta chain",
  "term_label": "Unknown biological process",
  "gene": "UniProtKB:P13224",
  "term_id": "UNKNOWN:0002"
}